{
  "gene": "UniProtKB:Q8NBF2",
  "term_label": "Unknown molecular function",
  "gene_symbol": "NHLRC2",
  "gene_name": "NHL repeat-containing protein 2",
  "term_id": "UNKNOWN:0001"
}